{
  "term_label": "Unknown molecular function",
  "term_id": "UNKNOWN:0001",
  "gene_symbol": "LINC00575",
  "gene_name": "Putative uncharacterized protein encoded by LINC00575",
  "gene": "UniProtKB:Q6W349"
}